{
  "gene_symbol": "KIF1B",
  "term_id": "GO:0005871",
  "gene": "UniProtKB:O60333",
  "term_label": "kinesin complex",
  "gene_name": "Kinesin-like protein KIF1B"
}